cellular response to nitrosative stress [GO:0071500] (biological process) Definition: Any process that results in a change in state or activity of a cell (in terms of movement, secretion, enzyme production, gene expression, etc.) as a result of a nitrosative stress stimulus. Nitrosative stress is a state often resulting from exposure to high levels of nitric oxide (NO) or the highly reactive oxidant peroxynitrite, which is produced following interaction of NO with superoxide anions. Subtypes: intrinsic apoptotic signaling pathway in response to nitrosative stress [GO:1990442] Relationships: is a type of response to nitrosative stress [GO:0051409]; is a type of cellular response to chemical stress [GO:0062197] Sources: GOC:mah